{
  "term_id": "GO:0005886",
  "term_label": "plasma membrane",
  "gene_name": "Bis(5'-adenosyl)-triphosphatase",
  "gene": "UniProtKB:P49789",
  "gene_symbol": "FHIT"
}